{
  "term_id": "GO:0031681",
  "term_label": "G-protein beta-subunit binding",
  "gene": "UniProtKB:Q9UBI6",
  "gene_symbol": "GNG12",
  "gene_name": "Guanine nucleotide-binding protein G(I)_G(S)_G(O) subunit gamma-12"
}